{
  "term_label": "DNA-binding transcription repressor activity, RNA polymerase II-specific",
  "gene": "UniProtKB:P41182",
  "gene_symbol": "BCL6",
  "gene_name": "B-cell lymphoma 6 protein",
  "term_id": "GO:0001227"
}